fungal-type vacuole lumen [GO:0000328] (cellular component) Sources: GOC:krc, GOC:mtg_sensu Definition: The volume enclosed within the vacuolar membrane of a vacuole, the shape of which correlates with cell cycle phase. An example of this structure is found in Saccharomyces cerevisiae. Also known as: lumen of vacuole with cell cycle-correlated morphology Relationships: is a type of vacuolar lumen [GO:0005775]; is part of fungal-type vacuole [GO:0000324]